low-affinity ferric iron ion transmembrane transporter activity [GO:0015090] (MF) Sources: TC:9.A.9.1.1 Also known as: low affinity iron ion transmembrane transporter activity, low affinity iron transporter activity Definition: Enables the transfer of a solute or solutes from one side of a membrane to the other according to the reaction: Fe2+(out) = Fe2+(in). In low-affinity transport the transporter is able to bind the solute only if it is present at very high concentrations. Relationships: is a type of ferric iron transmembrane transporter activity [GO:0015091]